positive regulation of mitotic metaphase/anaphase transition [GO:0045842] (biological process) Relationships: is a type of regulation of mitotic metaphase/anaphase transition [GO:0030071]; is a type of positive regulation of mitotic nuclear division [GO:0045840]; is a type of positive regulation of mitotic sister chromatid separation [GO:1901970]; is a type of positive regulation of mitotic cell cycle phase transition [GO:1901992]; is a type of positive regulation of metaphase/anaphase transition of cell cycle [GO:1902101]; positively regulates metaphase/anaphase transition of mitotic cell cycle [GO:0007091] Sources: GOC:go_curators Definition: Any process that activates or increases the frequency, rate or extent of the cell cycle process in which a cell progresses from metaphase to anaphase during mitosis, triggered by the activation of the anaphase promoting complex by Cdc20/Sleepy homolog which results in the degradation of Securin. Subtypes: GO:0140499 Also known as: up regulation of mitotic metaphase/anaphase transition, up-regulation of mitotic metaphase/anaphase transition, upregulation of mitotic metaphase/anaphase transition, activation of mitotic metaphase/anaphase transition, stimulation of mitotic metaphase/anaphase transition